symbiont-mediated perturbation of host cell endomembrane system [GO:0052025] (biological process) Relationships: is a type of GO:0141171 Definition: The process in which an organism effects a change that impairs the structure or function of the host endomembrane system. The host is defined as the larger of the organisms involved in a symbiotic interaction. Sources: GOC:mtg_pamgo_17jul06 Also known as: disruption by symbiont of host cell membrane, modification by symbiont of host cell membrane, symbiont-mediated disruption of host cell membrane, symbiont-mediated perturbation of host cell membrane